negative regulation of secondary metabolite biosynthetic process [GO:1900377] (biological process) Subtypes: negative regulation of melanin biosynthetic process [GO:0048022], negative regulation of aflatoxin biosynthetic process [GO:1900178], negative regulation of penicillin biosynthetic process [GO:1900197], GO:1900380, GO:1900627, GO:1900650, GO:1900653, negative regulation of diorcinol biosynthetic process [GO:1900656], negative regulation of emericellamide biosynthetic process [GO:1900659], negative regulation of emodin biosynthetic process [GO:1900665], negative regulation of endocrocin biosynthetic process [GO:1900668], negative regulation of fumonisin biosynthetic process [GO:1900684], negative regulation of gerfelin biosynthetic process [GO:1900687], negative regulation of gliotoxin biosynthetic process [GO:1900690], negative regulation of (+)-kotanin biosynthetic process [GO:1900693], negative regulation of N',N'',N'''-triacetylfusarinine C biosynthetic process [GO:1900696], negative regulation of o-orsellinic acid biosynthetic process [GO:1900699], negative regulation of orcinol biosynthetic process [GO:1900702], negative regulation of siderophore biosynthetic process [GO:1900705], GO:1900708, negative regulation of tensidol B biosynthetic process [GO:1900711], negative regulation of violaceol I biosynthetic process [GO:1900714], negative regulation of violaceol II biosynthetic process [GO:1900717], negative regulation of polyketide biosynthetic process [GO:1900733], negative regulation of sterigmatocystin biosynthetic process [GO:1900760], negative regulation of ergot alkaloid biosynthetic process [GO:1900823], negative regulation of emericellin biosynthetic process [GO:1900835], negative regulation of helvolic acid biosynthetic process [GO:1900841], negative regulation of monodictyphenone biosynthetic process [GO:1900844], negative regulation of cordyol C biosynthetic process [GO:1900862], negative regulation of syringal lignin biosynthetic process [GO:1901429], negative regulation of sinapate ester biosynthetic process [GO:1903086] Relationships: is a type of negative regulation of biosynthetic process [GO:0009890]; is a type of regulation of secondary metabolite biosynthetic process [GO:1900376]; negatively regulates GO:0044550 Sources: GOC:TermGenie, GOC:di Also known as: down regulation of secondary metabolite biosynthesis, down regulation of secondary metabolite biosynthetic process, down-regulation of secondary metabolite biosynthesis, down-regulation of secondary metabolite biosynthetic process, downregulation of secondary metabolite biosynthesis, downregulation of secondary metabolite biosynthetic process, inhibition of secondary metabolite biosynthesis, negative regulation of secondary metabolite biosynthesis, inhibition of secondary metabolite biosynthetic process Definition: Any process that stops, prevents or reduces the frequency, rate or extent of secondary metabolite biosynthetic process.